{
  "gene": "UniProtKB:Q1EHB4",
  "gene_symbol": "SLC5A12",
  "gene_name": "Sodium-coupled monocarboxylate transporter 2",
  "term_label": "symporter activity",
  "term_id": "GO:0015293"
}